{
  "term_id": "GO:0005886",
  "gene_symbol": "GPR37",
  "term_label": "plasma membrane",
  "gene": "UniProtKB:O15354",
  "gene_name": "Prosaposin receptor GPR37"
}